{
  "term_id": "UNKNOWN:0002",
  "term_label": "Unknown biological process",
  "gene": "UniProtKB:H3BTG2",
  "gene_symbol": "TEX46",
  "gene_name": "Testis-expressed protein 46"
}